chloroplastic endopeptidase Clp complex [GO:0009840] (cellular component) Relationships: is a type of endopeptidase Clp complex [GO:0009368]; is part of chloroplast stroma [GO:0009570] Sources: GOC:mah Definition: A Clp endopeptidase complex located in the chloroplast.